{
  "gene_name": "Dolichol-phosphate mannosyltransferase subunit 1",
  "term_label": "protein O-linked glycosylation via mannose",
  "gene_symbol": "DPM1",
  "term_id": "GO:0035269",
  "gene": "UniProtKB:O60762"
}